{
  "gene": "UniProtKB:P54219",
  "term_label": "terminal bouton",
  "gene_symbol": "SLC18A1",
  "gene_name": "Chromaffin granule amine transporter",
  "term_id": "GO:0043195"
}